{
  "term_id": "GO:0023026",
  "gene_name": "HLA class II histocompatibility antigen, DR beta 5 chain",
  "gene": "UniProtKB:Q30154",
  "gene_symbol": "HLA-DRB5",
  "term_label": "MHC class II protein complex binding"
}